positive regulation of intrinsic apoptotic signaling pathway by p53 class mediator [GO:1902255] (biological process) Definition: Any process that activates or increases the frequency, rate or extent of intrinsic apoptotic signaling pathway by p53 class mediator. References: PMID:15705871 Sources: GOC:BHF, GOC:TermGenie, GOC:mtg_apoptosis, GOC:rl Also known as: positive regulation of intrinsic apoptotic signaling pathway by signal transduction by p53 class mediator, up regulation of intrinsic apoptotic signaling pathway by p53 class mediator, up regulation of intrinsic apoptotic signaling pathway by signal transduction by p53 class mediator, up-regulation of intrinsic apoptotic signaling pathway by p53 class mediator, up-regulation of intrinsic apoptotic signaling pathway by signal transduction by p53 class mediator, upregulation of intrinsic apoptotic signaling pathway by p53 class mediator, upregulation of intrinsic apoptotic signaling pathway by signal transduction by p53 class mediator, activation of intrinsic apoptotic signaling pathway by p53 class mediator, activation of intrinsic apoptotic signaling pathway by signal transduction by p53 class mediator, activation of signal transduction by p53 class mediator resulting in induction of apoptosis, positive regulation of signal transduction by p53 class mediator resulting in induction of apoptosis, up regulation of signal transduction by p53 class mediator resulting in induction of apoptosis, up-regulation of signal transduction by p53 class mediator resulting in induction of apoptosis, upregulation of signal transduction by p53 class mediator resulting in induction of apoptosis Relationships: is a type of positive regulation of signal transduction by p53 class mediator [GO:1901798]; is a type of regulation of intrinsic apoptotic signaling pathway by p53 class mediator [GO:1902253]; is a type of GO:2001244; positively regulates intrinsic apoptotic signaling pathway by p53 class mediator [GO:0072332] Subtypes: positive regulation of intrinsic apoptotic signaling pathway in response to DNA damage by p53 class mediator [GO:1902167], positive regulation of intrinsic apoptotic signaling pathway in response to osmotic stress by p53 class mediator [GO:1902240]